CCL21-activated CCR7 signaling pathway [GO:0038120] (biological process) References: PMID:15059845 Sources: GOC:nhn, GOC:signaling Also known as: CCL21-activated CCR7 signalling pathway Definition: The series of molecular signals initiated by the binding of the C-C chemokine CCL21 to a C-C chemokine type 7 receptor (CCR7) on the surface of a target cell, and ending with the regulation of a downstream cellular process, e.g. transcription. Relationships: is a type of chemokine (C-C motif) ligand 21 signaling pathway [GO:0038116]; is a type of C-C chemokine receptor CCR7 signaling pathway [GO:0038118]